{
  "term_id": "GO:0005543",
  "term_label": "phospholipid binding",
  "gene_name": "Group 10 secretory phospholipase A2",
  "gene_symbol": "PLA2G10",
  "gene": "UniProtKB:O15496"
}